{
  "gene": "UniProtKB:C9JVW0",
  "gene_name": "Putative transmembrane protein INAFM1",
  "gene_symbol": "INAFM1",
  "term_label": "Unknown biological process",
  "term_id": "UNKNOWN:0002"
}